{
  "gene": "UniProtKB:Q86WT1",
  "term_label": "axonemal microtubule",
  "gene_symbol": "IFT70A",
  "term_id": "GO:0005879",
  "gene_name": "Intraflagellar transport protein 70A"
}